{
  "gene_symbol": "B3GNT5",
  "term_id": "GO:0000139",
  "term_label": "Golgi membrane",
  "gene_name": "Lactosylceramide 1,3-N-acetyl-beta-D-glucosaminyltransferase",
  "gene": "UniProtKB:Q9BYG0"
}